{
  "term_label": "vascular endothelial growth factor receptor activity",
  "gene_name": "Vascular endothelial growth factor receptor 2",
  "term_id": "GO:0005021",
  "gene": "UniProtKB:P35968",
  "gene_symbol": "KDR"
}